{
  "term_id": "UNKNOWN:0002",
  "gene": "UniProtKB:O14792",
  "gene_name": "Heparan sulfate glucosamine 3-O-sulfotransferase 1",
  "term_label": "Unknown biological process",
  "gene_symbol": "HS3ST1"
}